cell-matrix adhesion involved in ameboidal cell migration [GO:0003366] (biological process) Subtypes: cell-matrix adhesion involved in mesendodermal cell migration [GO:0003368] Relationships: is a type of cell-matrix adhesion [GO:0007160]; is part of ameboidal-type cell migration [GO:0001667] Sources: GOC:ascb_2009, GOC:dph, GOC:tb Definition: The binding of a cell to the extracellular matrix that contributes to the directed movement of an ameboid cell.